{
  "gene_name": "Alpha-crystallin A chain",
  "gene": "UniProtKB:P02489",
  "term_id": "GO:0005737",
  "term_label": "cytoplasm",
  "gene_symbol": "CRYAA"
}